{
  "gene": "UniProtKB:Q9Y2B5",
  "gene_name": "VPS9 domain-containing protein 1",
  "term_id": "GO:0005829",
  "term_label": "cytosol",
  "gene_symbol": "VPS9D1"
}